mannose-specific flocculation [GO:0036350] (biological process) Definition: The non-sexual aggregation of single-celled organisms mediated by the binding of cell wall proteins on one cell to mannose residues on the other. References: PMID:9851992 Sources: GOC:vw Also known as: cell-cell adhesion involved in mannose-specific flocculation Relationships: is a type of flocculation [GO:0000128]; has part D-mannose binding [GO:0005537]